response to fluoxetine [GO:0014076] (biological process) Note: Note that this term is in the subset of terms that should not be used for direct manual annotation of gene products. Direct annotations to this term may be amended during annotation QC. Relationships: is_a response to antidepressant [GO:0036276] Definition: Any process that results in a change in state or activity of a cell or an organism (in terms of movement, secretion, enzyme production, gene expression, etc.) as a result of a fluoxetine stimulus. Fluoxetine increases the extracellular level of the neurotransmitter serotonin by inhibiting its reuptake into the presynaptic cell, increasing the level of serotonin available to bind to the postsynaptic receptor. Sources: GOC:ef, GOC:pr Subtypes: cellular response to fluoxetine [GO:0071411] Also known as: response to SSRI, response to selective serotonin reuptake inhibitor